Delta1 complex [GO:0070763] (cellular component) Definition: A protein complex that consists of homodimer of the Notch ligand Delta1. Also known as: Delta1 homodimer complex References: PMID:12794186 Relationships: is_a plasma membrane protein complex [GO:0098797]